{
  "gene": "UniProtKB:Q5VU43",
  "gene_name": "Myomegalin",
  "term_label": "molecular adaptor activity",
  "gene_symbol": "PDE4DIP",
  "term_id": "GO:0060090"
}